{
  "term_id": "GO:0005686",
  "gene": "UniProtKB:Q9Y388",
  "gene_symbol": "RBMX2",
  "term_label": "U2 snRNP",
  "gene_name": "RNA-binding motif protein, X-linked 2"
}